titin binding [GO:0031432] (molecular function) Definition: Binding to titin, any of a family of giant proteins found in striated and smooth muscle. In striated muscle, single titin molecules span half the sarcomere, with their N- and C-termini in the Z-disc and M-line, respectively. References: PMID:10481174 Sources: GOC:mah Relationships: is a type of GO:0008092